{
  "gene_name": "Chorion-specific transcription factor GCMa",
  "gene": "UniProtKB:Q9NP62",
  "term_id": "GO:0005634",
  "gene_symbol": "GCM1",
  "term_label": "nucleus"
}